{
  "term_id": "GO:0005634",
  "term_label": "nucleus",
  "gene": "UniProtKB:Q99676",
  "gene_name": "Zinc finger protein 184",
  "gene_symbol": "ZNF184"
}